{
  "gene_symbol": "RAD51B",
  "term_id": "GO:0003697",
  "term_label": "single-stranded DNA binding",
  "gene": "UniProtKB:O15315",
  "gene_name": "DNA repair protein RAD51 homolog 2"
}